{
  "gene": "UniProtKB:Q9BSB4",
  "term_label": "phagophore assembly site",
  "gene_name": "Autophagy-related protein 101",
  "gene_symbol": "ATG101",
  "term_id": "GO:0000407"
}